{
  "gene_name": "Krueppel-like factor 2",
  "term_id": "GO:0006357",
  "gene": "UniProtKB:Q9Y5W3",
  "gene_symbol": "KLF2",
  "term_label": "regulation of transcription by RNA polymerase II"
}